regulation of stem cell proliferation [GO:0072091] (biological process) Definition: Any process that modulates the frequency, rate or extent of stem cell proliferation. A stem cell is a cell that retains the ability to divide and proliferate throughout life to provide progenitor cells that can differentiate into specialized cells. Relationships: is a type of regulation of cell population proliferation [GO:0042127]; regulates stem cell proliferation [GO:0072089] Sources: GOC:mtg_kidney_jan10 Subtypes: regulation of hematopoietic stem cell proliferation [GO:1902033], GO:1902460, negative regulation of stem cell proliferation [GO:2000647], positive regulation of stem cell proliferation [GO:2000648]